{
  "gene_symbol": "SLC66A2",
  "term_label": "trans-Golgi network membrane",
  "gene": "UniProtKB:Q8N2U9",
  "gene_name": "Solute carrier family 66 member 2",
  "term_id": "GO:0032588"
}